establishment of cell polarity involved in growth plate cartilage chondrocyte division [GO:0003424] (BP) Also known as: growth plate cartilage chondrocyte polarization Relationships: is a type of establishment of planar polarity [GO:0001736]; is a type of establishment of cell polarity [GO:0030010]; is part of growth plate cartilage chondrocyte division [GO:0003423] Sources: GOC:ascb_2009, GOC:dph, GOC:tb Definition: The cellular process that results in the specification, formation or maintenance of anisotropic intracellular organization that results in the directional division of a growth plate cartilage chondrocyte.